{
  "term_label": "Unknown cellular component",
  "gene_name": "Protein LSM12",
  "gene": "UniProtKB:Q3MHD2",
  "term_id": "UNKNOWN:0003",
  "gene_symbol": "LSM12"
}